{
  "gene": "UniProtKB:Q9BWN1",
  "gene_name": "Proline-rich protein 14",
  "term_id": "GO:0005654",
  "term_label": "nucleoplasm",
  "gene_symbol": "PRR14"
}